{
  "gene_symbol": "CFAP45",
  "term_id": "UNKNOWN:0001",
  "term_label": "Unknown molecular function",
  "gene": "UniProtKB:Q9UL16",
  "gene_name": "Cilia- and flagella-associated protein 45"
}